{
  "gene_name": "DNA damage-inducible transcript 4-like protein",
  "gene_symbol": "DDIT4L",
  "term_id": "UNKNOWN:0003",
  "gene": "UniProtKB:Q96D03",
  "term_label": "Unknown cellular component"
}